{
  "term_label": "cytosol",
  "term_id": "GO:0005829",
  "gene_name": "Rho-related GTP-binding protein Rho6",
  "gene": "UniProtKB:Q92730",
  "gene_symbol": "RND1"
}